slit diaphragm assembly [GO:0036060] (biological process) Definition: The aggregation, arrangement and bonding together of a set of components to form a slit diaphragm, specialized cell-cell junction found between the interdigitating foot processes of the glomerular epithelium (the podocytes) in the vertebrate kidney, which is adapted for facilitating glomerular filtration. Relationships: is a type of filtration diaphragm assembly [GO:0036058] References: PMID:20633639 Sources: GOC:mtg_kidney_jan10, GOC:rph